{
  "term_label": "regulation of insulin-like growth factor receptor signaling pathway",
  "gene_name": "Insulin-like growth factor-binding protein 6",
  "gene_symbol": "IGFBP6",
  "gene": "UniProtKB:P24592",
  "term_id": "GO:0043567"
}